{
  "gene": "UniProtKB:Q8IUZ5",
  "term_label": "Unknown biological process",
  "gene_symbol": "PHYKPL",
  "gene_name": "5-phosphohydroxy-L-lysine phospho-lyase",
  "term_id": "UNKNOWN:0002"
}